{
  "gene_name": "Retinoic acid receptor beta",
  "gene_symbol": "RARB",
  "gene": "UniProtKB:P10826",
  "term_label": "positive regulation of transcription by RNA polymerase II",
  "term_id": "GO:0045944"
}